effector-mediated suppression of host pattern-triggered immunity signaling [GO:0140423] (biological process) Also known as: effector-mediated suppression of host PRR signaling, effector-mediated suppression of host PRR signalling, effector-mediated suppression of host pattern recognition receptor signaling, effector-mediated suppression of PTI signalling, effector-mediated suppression of pattern-triggered immunity signaling Relationships: is_a GO:0052034 References: PMID:30584105 Definition: A process mediated by a molecule secreted by a symbiont that results in the suppression of a pattern-triggered immunity PTI signaling pathway. PTI signaling pathways are found in plants.